{
  "term_id": "GO:0003713",
  "gene_name": "Homeodomain-interacting protein kinase 2",
  "gene_symbol": "HIPK2",
  "term_label": "transcription coactivator activity",
  "gene": "UniProtKB:Q9H2X6"
}